tRNA-splicing ligase complex [GO:0072669] (cellular component) Also known as: tRNA splicing ligase complex Relationships: is a type of intracellular protein-containing complex [GO:0140535]; is a type of catalytic complex [GO:1902494] References: PMID:21311021 Sources: GOC:sp Definition: A protein complex that catalyzes the ligation of cleaved pre-tRNAs by directly joining spliced tRNA halves to mature-sized tRNAs by incorporating the precursor-derived splice junction phosphate into the mature tRNA as a canonical 3',5'-phosphodiester.